{
  "gene_name": "Marginal zone B- and B1-cell-specific protein",
  "gene_symbol": "MZB1",
  "term_label": "extracellular region",
  "gene": "UniProtKB:Q8WU39",
  "term_id": "GO:0005576"
}